{
  "term_label": "transmembrane signaling receptor activity",
  "gene": "UniProtKB:Q9Y5Y7",
  "term_id": "GO:0004888",
  "gene_symbol": "LYVE1",
  "gene_name": "Lymphatic vessel endothelial hyaluronic acid receptor 1"
}